{
  "gene": "UniProtKB:O75143",
  "gene_symbol": "ATG13",
  "term_id": "GO:0034497",
  "gene_name": "Autophagy-related protein 13",
  "term_label": "protein localization to phagophore assembly site"
}